negative regulation of ovulation [GO:0060280] (biological process) Definition: Any process that stops, prevents, or reduces the frequency, rate or extent of ovulation, the release of a mature ovum/oocyte from an ovary. Relationships: is a type of negative regulation of multicellular organismal process [GO:0051241]; is a type of GO:0060278; is a type of negative regulation of reproductive process [GO:2000242]; negatively regulates ovulation [GO:0030728] Sources: GOC:dph, GOC:kmv, GOC:tb